{
  "gene": "UniProtKB:O75969",
  "term_label": "intracellular protein localization",
  "gene_name": "A-kinase anchor protein 3",
  "term_id": "GO:0008104",
  "gene_symbol": "AKAP3"
}